{
  "term_label": "D5 dopamine receptor binding",
  "gene": "UniProtKB:Q03113",
  "gene_name": "Guanine nucleotide-binding protein subunit alpha-12",
  "gene_symbol": "GNA12",
  "term_id": "GO:0031752"
}